{
  "gene_symbol": "ALDH5A1",
  "gene": "UniProtKB:P51649",
  "gene_name": "Succinate-semialdehyde dehydrogenase, mitochondrial",
  "term_id": "GO:0009450",
  "term_label": "gamma-aminobutyric acid catabolic process"
}